{
  "gene_symbol": "SCNN1G",
  "gene_name": "Amiloride-sensitive sodium channel subunit gamma",
  "gene": "UniProtKB:P51170",
  "term_label": "ligand-gated sodium channel activity",
  "term_id": "GO:0015280"
}